tricarboxylic acid metabolic process [GO:0072350] (biological process) Definition: The chemical reactions and pathways involving dicarboxylic acids, any organic acid containing three carboxyl (COOH) groups or anions (COO-). Sources: GOC:mah Also known as: tricarboxylic acid metabolism Relationships: is a type of carboxylic acid metabolic process [GO:0019752] Subtypes: argininosuccinate metabolic process [GO:0000053], citrate metabolic process [GO:0006101], isocitrate metabolic process [GO:0006102], tricarboxylic acid biosynthetic process [GO:0072351], GO:0072352, sarcinapterin metabolic process [GO:1900867]